regulation of L-glutamine import across plasma membrane [GO:1901034] (biological process) Definition: Any process that modulates the frequency, rate or extent of L-glutamine import into cell. Subtypes: negative regulation of L-glutamine import across plasma membrane [GO:1901035], positive regulation of L-glutamine import across plasma membrane [GO:1901036] Sources: GOC:TermGenie Also known as: regulation of L-glutamine import, regulation of L-glutamine uptake Relationships: is a type of regulation of amino acid import across plasma membrane [GO:0010958]; is a type of regulation of glutamine transport [GO:2000485]; regulates L-glutamine import across plasma membrane [GO:1903803]